{
  "gene_name": "Cytoskeleton-associated protein 2-like",
  "gene_symbol": "CKAP2L",
  "gene": "UniProtKB:Q8IYA6",
  "term_label": "Unknown biological process",
  "term_id": "UNKNOWN:0002"
}